specification of segmental identity, head [GO:0007380] (BP) Definition: The specification of the characteristic structures of the head segments following establishment of segment boundaries. Identity is considered to be the aggregate of characteristics by which a structure is recognized. Subtypes: GO:0007381, GO:0007382, GO:0007383, specification of segmental identity, intercalary segment [GO:0035291], specification of segmental identity, mandibular segment [GO:0042305] Relationships: is a type of segment specification [GO:0007379]; is part of GO:0035287 Sources: ISBN:0878932437